{
  "gene": "UniProtKB:Q9BQI9",
  "term_label": "aspartic-type endopeptidase activity",
  "term_id": "GO:0004190",
  "gene_name": "Nuclear receptor-interacting protein 2",
  "gene_symbol": "NRIP2"
}